{
  "term_id": "GO:0050839",
  "gene_symbol": "PCDHB1",
  "term_label": "cell adhesion molecule binding",
  "gene": "UniProtKB:Q9Y5F3",
  "gene_name": "Protocadherin beta-1"
}